{
  "gene_name": "Ras GTPase-activating protein nGAP",
  "term_label": "regulation of intracellular signal transduction",
  "term_id": "GO:1902531",
  "gene": "UniProtKB:Q9UJF2",
  "gene_symbol": "RASAL2"
}